{
  "gene": "UniProtKB:O43603",
  "term_label": "galanin-activated signaling pathway",
  "term_id": "GO:0090663",
  "gene_name": "Galanin receptor type 2",
  "gene_symbol": "GALR2"
}